{
  "gene_name": "Mothers against decapentaplegic homolog 6",
  "gene_symbol": "SMAD6",
  "term_label": "I-SMAD binding",
  "term_id": "GO:0070411",
  "gene": "UniProtKB:O43541"
}